{
  "term_label": "cytoplasm",
  "gene": "UniProtKB:Q08752",
  "term_id": "GO:0005737",
  "gene_name": "Peptidyl-prolyl cis-trans isomerase D",
  "gene_symbol": "PPID"
}